zeatin 9-aminocarboxyethyltransferase activity [GO:0050447] (molecular function) Definition: Catalysis of the reaction: O-acetyl-L-serine + zeatin = L-lupinate + acetate + H+. Sources: EC:2.5.1.50, RHEA:17333 Also known as: beta-(9-cytokinin)-alanine synthase activity, 3-O-acetyl-L-serine:zeatin 2-amino-2-carboxyethyltransferase activity, O-acetyl-L-serine acetate-lyase (adding N(6)-substituted adenine) activity, O-acetyl-L-serine acetate-lyase (adding N6-substituted adenine), O3-acetyl-L-serine:zeatin 2-amino-2-carboxyethyltransferase activity, beta-(9-cytokinin)alanine synthase activity, lupinate synthetase activity, lupinic acid synthase activity, lupinic acid synthetase activity Relationships: is a type of transferase activity, transferring alkyl or aryl (other than methyl) groups [GO:0016765]